positive regulation of triglyceride transport [GO:1905885] (biological process) Relationships: is a type of positive regulation of acylglycerol transport [GO:1901508]; is a type of GO:1905883; positively regulates GO:0034197 References: PMID:25849533 Sources: GOC:TermGenie, GO_REF:0000058 Definition: Any process that activates or increases the frequency, rate or extent of triglyceride transport. Also known as: positive regulation of triacylglycerol transport, up regulation of triacylglycerol transport, up regulation of triglyceride transport, up-regulation of triacylglycerol transport, up-regulation of triglyceride transport, upregulation of triacylglycerol transport, upregulation of triglyceride transport, activation of triacylglycerol transport, activation of triglyceride transport